{
  "gene": "UniProtKB:Q8IZ40",
  "gene_name": "REST corepressor 2",
  "gene_symbol": "RCOR2",
  "term_label": "histone deacetylase complex",
  "term_id": "GO:0000118"
}